mesoderm development [GO:0007498] (biological process) Relationships: is a type of tissue development [GO:0009888] Definition: The process whose specific outcome is the progression of the mesoderm over time, from its formation to the mature structure. The mesoderm is the middle germ layer that develops into muscle, bone, cartilage, blood and connective tissue. Regulation: RO_0002211 by regulation of mesoderm development [GO:2000380]; negatively regulated by GO:2000381; positively regulated by positive regulation of mesoderm development [GO:2000382] Sources: GOC:dph, GOC:tb Subtypes: GO:0007506, axial mesoderm development [GO:0048318], paraxial mesoderm development [GO:0048339], lateral mesoderm development [GO:0048368], intermediate mesoderm development [GO:0048389]